type III site-specific deoxyribonuclease activity [GO:0015668] (molecular function) Definition: Catalysis of the endonucleolytic cleavage of DNA to give double-stranded fragments with terminal 5'-phosphates. ATP hydrolysis is required. Cleavage is dependent on the presence of two copies of a specific recognition sequence in an inverse orientation in the DNA. Cleavage occurs at a specific distance from one of the recognition sites. Relationships: is a type of restriction endodeoxyribonuclease activity [GO:0015666]; is a type of GO:0016888 Also known as: type III restriction enzyme activity References: PMID:12654995 Sources: EC:3.1.21.5